galactose-6-sulfurylase activity [GO:0033844] (molecular function) Definition: Catalysis of the elimination of sulfate from the D-galactose 6-sulfate residues of porphyran, producing 3,6-anhydrogalactose residues. Sources: EC:2.5.1.5 Also known as: D-galactose-6-sulfate:alkyltransferase (cyclizing) activity, galactose 6-sulfatase activity, galactose-6-sulfatase activity, porphyran sulfatase activity Relationships: is a type of transferase activity, transferring alkyl or aryl (other than methyl) groups [GO:0016765]